{
  "gene": "UniProtKB:P00813",
  "term_label": "cytosol",
  "gene_symbol": "ADA",
  "term_id": "GO:0005829",
  "gene_name": "Adenosine deaminase"
}